{
  "gene_symbol": "IGHV3-73",
  "term_id": "UNKNOWN:0003",
  "gene_name": "Immunoglobulin heavy variable 3-73",
  "term_label": "Unknown cellular component",
  "gene": "UniProtKB:A0A0B4J1V6"
}